{
  "gene_symbol": "ZNF131",
  "term_label": "DNA-binding transcription repressor activity, RNA polymerase II-specific",
  "term_id": "GO:0001227",
  "gene_name": "Zinc finger protein 131",
  "gene": "UniProtKB:P52739"
}